{
  "term_id": "GO:0046703",
  "gene": "UniProtKB:Q9BZM6",
  "gene_name": "UL16-binding protein 1",
  "gene_symbol": "ULBP1",
  "term_label": "natural killer cell lectin-like receptor binding"
}